{
  "gene_symbol": "GOLGB1",
  "term_id": "GO:0005793",
  "gene": "UniProtKB:Q14789",
  "gene_name": "Golgin subfamily B member 1",
  "term_label": "endoplasmic reticulum-Golgi intermediate compartment"
}